{
  "term_id": "GO:0005615",
  "gene_symbol": "PPBP",
  "gene_name": "Platelet basic protein",
  "gene": "UniProtKB:P02775",
  "term_label": "extracellular space"
}